{
  "gene": "UniProtKB:P11831",
  "term_id": "GO:0000981",
  "term_label": "DNA-binding transcription factor activity, RNA polymerase II-specific",
  "gene_symbol": "SRF",
  "gene_name": "Serum response factor"
}